{
  "term_id": "GO:0031768",
  "gene": "UniProtKB:Q9UBU3",
  "gene_symbol": "GHRL",
  "term_label": "ghrelin receptor binding",
  "gene_name": "Appetite-regulating hormone"
}